{
  "gene_symbol": "TEKT1",
  "gene_name": "Tektin-1",
  "gene": "UniProtKB:Q969V4",
  "term_id": "GO:0060294",
  "term_label": "cilium movement involved in cell motility"
}